riboflavin metabolic process [GO:0006771] (biological process) Definition: The chemical reactions and pathways involving riboflavin (vitamin B2), the precursor for the coenzymes flavin mononucleotide (FMN) and flavin adenine dinucleotide (FAD). Also known as: riboflavin metabolism, vitamin B2 metabolic process, vitamin B2 metabolism, vitamin G metabolic process, vitamin G metabolism Subtypes: riboflavin biosynthetic process [GO:0009231], riboflavin catabolic process [GO:0009232] References: PMID:11153262, PMID:24764086 Sources: GOC:jl Relationships: is a type of flavin-containing compound metabolic process [GO:0042726]